{
  "gene_symbol": "AGPAT5",
  "gene_name": "1-acyl-sn-glycerol-3-phosphate acyltransferase epsilon",
  "term_id": "GO:0012505",
  "gene": "UniProtKB:Q9NUQ2",
  "term_label": "endomembrane system"
}